{
  "term_id": "GO:0004016",
  "gene_symbol": "ADCY1",
  "gene": "UniProtKB:Q08828",
  "term_label": "adenylate cyclase activity",
  "gene_name": "Adenylate cyclase type 1"
}